wall teichoic acid catabolic process [GO:0070399] (BP) Relationships: is a type of cell wall macromolecule catabolic process [GO:0016998]; is a type of teichoic acid catabolic process [GO:0070393] References: PMID:14665680 Sources: GOC:add Also known as: wall teichoic acid breakdown, wall teichoic acid catabolism, wall teichoic acid degradation Definition: The chemical reactions and pathways resulting in the breakdown of wall teichoic acid, which is a major component of the cell wall of Gram-positive bacteria and typically consists of a polymer of glycerol-phosphate or ribitol-phosphate to which are attached glycosyl and D-alanyl ester residues and which is covalently linked to peptidoglycan.